{
  "gene_symbol": "IDUA",
  "term_id": "GO:0003940",
  "gene": "UniProtKB:P35475",
  "gene_name": "Alpha-L-iduronidase",
  "term_label": "L-iduronidase activity"
}